loganate O-methyltransferase activity [GO:0030749] (molecular function) Sources: EC:2.1.1.50 Definition: Catalysis of the reaction: S-adenosyl-L-methionine + loganate = S-adenosyl-L-homocysteine + loganin. Relationships: is a type of S-adenosylmethionine-dependent methyltransferase activity [GO:0008757] Also known as: S-adenosyl-L-methionine:loganate 11-O-methyltransferase activity, S-adenosyl-L-methionine:loganic acid methyltransferase activity, loganate methyltransferase activity